{
  "gene_symbol": "SKAP1",
  "gene_name": "Src kinase-associated phosphoprotein 1",
  "term_label": "plasma membrane",
  "gene": "UniProtKB:Q86WV1",
  "term_id": "GO:0005886"
}